{
  "gene_name": "Olfactory receptor 5AC1",
  "term_id": "UNKNOWN:0002",
  "gene": "UniProtKB:P0C628",
  "gene_symbol": "OR5AC1",
  "term_label": "Unknown biological process"
}